{
  "term_label": "circadian regulation of gene expression",
  "gene_name": "Circadian-associated transcriptional repressor",
  "gene": "UniProtKB:Q8N365",
  "gene_symbol": "CIART",
  "term_id": "GO:0032922"
}